epidermal cell fate specification [GO:0009957] (biological process) Definition: The process in which a cell becomes capable of differentiating autonomously into an epidermal cell in an environment that is neutral with respect to the developmental pathway; upon specification, the cell fate can be reversed. Sources: GOC:mtg_sensu, GOC:sm Also known as: hypodermal cell fate specification Relationships: is a type of cell fate specification [GO:0001708]; is part of epidermal cell differentiation [GO:0009913] Subtypes: limb basal epidermal cell fate specification [GO:0060892], limb granular cell fate specification [GO:0060893], limb spinous cell fate specification [GO:0060894]